soft palate development [GO:0060023] (BP) Sources: GOC:dph, ISBN:0721662544 Definition: The biological process whose specific outcome is the progression of the soft palate from an initial condition to its mature state. This process begins with the formation of the structure and ends with the mature structure, whatever form that may be including its natural destruction. The soft palate is the posterior portion of the palate extending from the posterior edge of the hard palate. Relationships: is a type of GO:0048856; is part of secondary palate development [GO:0062009] Also known as: palatum molle development, velum palatum development